{
  "gene": "UniProtKB:Q02252",
  "term_id": "GO:0006210",
  "term_label": "thymine catabolic process",
  "gene_name": "Methylmalonate-semialdehyde dehydrogenase [acylating], mitochondrial",
  "gene_symbol": "ALDH6A1"
}